pollen aperture formation [GO:0062075] (biological process) References: PMID:30150313 Relationships: is a type of cellular component assembly involved in morphogenesis [GO:0010927]; is part of GO:0010208 Definition: The cellular component assembly process of forming pollen apertures, areas where exine is reduced or absent, in the pollen cell wall.